{
  "term_label": "Golgi membrane",
  "gene_symbol": "RAB2B",
  "gene": "UniProtKB:Q8WUD1",
  "gene_name": "Ras-related protein Rab-2B",
  "term_id": "GO:0000139"
}